{
  "term_id": "GO:0032088",
  "gene": "UniProtKB:P20749",
  "gene_name": "B-cell lymphoma 3 protein",
  "gene_symbol": "BCL3",
  "term_label": "negative regulation of NF-kappaB transcription factor activity"
}